TACC/TOG complex [GO:0070850] (cellular component) References: PMID:19606211 Sources: GOC:mah, GOC:vw Relationships: is a type of intracellular protein-containing complex [GO:0140535] Definition: A protein complex that contains the transforming acidic coiled coil (TACC) protein and the TOG protein (Mia1p/Alp7p and Alp14, respectively, in fission yeast), and is involved in microtubule array remodeling as cells progress through the cell cycle. The TACC/TOG complex is conserved in eukaryotes, associates with microtubules, and shuttles between the nucleus and the cytoplasm during interphase.